memory T cell extravasation [GO:0035683] (biological process) Relationships: is a type of T cell extravasation [GO:0072683] Also known as: memory T-cell extravasation Definition: The migration of a memory T cell from the blood vessels into the surrounding tissue. A memory T cell is a distinctly differentiated long-lived T cell that has the phenotype CD45RO-positive and CD127-positive. Sources: CL:0000813, GOC:BHF